adenylate cyclase activity [GO:0004016] (molecular function) Sources: EC:4.6.1.1 Definition: Catalysis of the reaction: ATP = 3',5'-cyclic AMP + diphosphate. Relationships: is a type of cyclase activity [GO:0009975]; is a type of phosphorus-oxygen lyase activity [GO:0016849] Also known as: adenylyl cyclase activity, 3',5'-cyclic AMP synthetase activity, ATP diphosphate-lyase (cyclizing) activity, ATP diphosphate-lyase (cyclizing; 3',5'-cyclic-AMP-forming) activity, ATP pyrophosphate-lyase activity, adenyl cyclase activity, adenylylcyclase activity, cAMP generating peptide activity Regulation: negatively regulated by GO:0007194; regulated by adenylate cyclase regulator activity [GO:0010854]; negatively regulated by GO:0010855; RO_0002213 by adenylate cyclase activator activity [GO:0010856]; regulated by regulation of adenylate cyclase activity [GO:0045761]; positively regulated by positive regulation of adenylate cyclase activity [GO:0045762] Subtypes: GO:0008294